{
  "gene_name": "Semaphorin-3C",
  "term_label": "positive regulation of cell migration",
  "term_id": "GO:0030335",
  "gene_symbol": "SEMA3C",
  "gene": "UniProtKB:Q99985"
}